{
  "gene": "UniProtKB:Q9UHA7",
  "gene_name": "Interleukin-36 alpha",
  "term_id": "GO:0005615",
  "gene_symbol": "IL36A",
  "term_label": "extracellular space"
}